{
  "gene_name": "DNA-directed RNA polymerase III subunit RPC6",
  "term_label": "RNA polymerase III complex",
  "gene_symbol": "POLR3F",
  "term_id": "GO:0005666",
  "gene": "UniProtKB:Q9H1D9"
}